pyrimidine nucleotide biosynthetic process [GO:0006221] (BP) Relationships: is a type of GO:0006220; is a type of nucleotide biosynthetic process [GO:0009165]; is a type of pyrimidine-containing compound biosynthetic process [GO:0072528] Regulation: regulated by regulation of pyrimidine nucleotide biosynthetic process [GO:1900397]; negatively regulated by negative regulation of pyrimidine nucleotide biosynthetic process [GO:1900398]; positively regulated by positive regulation of pyrimidine nucleotide biosynthetic process [GO:1900399] Subtypes: pyrimidine ribonucleotide biosynthetic process [GO:0009220], pyrimidine deoxyribonucleotide biosynthetic process [GO:0009221], pyrimidine nucleotide salvage [GO:0032262] Sources: GOC:go_curators, ISBN:0198506732 Also known as: pyrimidine nucleotide anabolism, pyrimidine nucleotide biosynthesis, pyrimidine nucleotide formation, pyrimidine nucleotide synthesis Definition: The chemical reactions and pathways resulting in the formation of a pyrimidine nucleotide, a compound consisting of nucleoside (a pyrimidine base linked to a deoxyribose or ribose sugar) esterified with a phosphate group at either the 3' or 5'-hydroxyl group of the sugar.